{
  "gene_symbol": "UNC93B1",
  "term_label": "toll-like receptor 3 signaling pathway",
  "term_id": "GO:0034138",
  "gene_name": "Protein unc-93 homolog B1",
  "gene": "UniProtKB:Q9H1C4"
}